{
  "gene_name": "Ceroid-lipofuscinosis neuronal protein 6",
  "gene": "UniProtKB:Q9NWW5",
  "term_label": "endoplasmic reticulum",
  "gene_symbol": "CLN6",
  "term_id": "GO:0005783"
}